budding cell isotropic bud growth [GO:0007119] (biological process) Sources: GOC:go_curators Definition: Unlocalized bud growth such that the entire surface of the bud expands evenly, in a cell that reproduces by budding. Also known as: isotropic bud growth Relationships: is a type of budding cell bud growth [GO:0007117]